negative regulation of interleukin-15 production [GO:0032698] (biological process) Also known as: down regulation of interleukin-15 production, down-regulation of interleukin-15 production, downregulation of interleukin-15 production, negative regulation of IL-15 production, inhibition of interleukin-15 production, negative regulation of interleukin-15 biosynthetic process Definition: Any process that stops, prevents, or reduces the frequency, rate, or extent of interleukin-15 production. Relationships: is a type of negative regulation of cytokine production [GO:0001818]; is a type of regulation of interleukin-15 production [GO:0032658]; RO_0002212 interleukin-15 production [GO:0032618] Sources: GOC:mah